{
  "term_label": "regulation of DNA-templated transcription",
  "term_id": "GO:0006355",
  "gene": "UniProtKB:Q8WYH8",
  "gene_name": "Inhibitor of growth protein 5",
  "gene_symbol": "ING5"
}